{
  "gene": "UniProtKB:Q8IV45",
  "gene_name": "UNC5C-like protein",
  "term_id": "UNKNOWN:0003",
  "gene_symbol": "UNC5CL",
  "term_label": "Unknown cellular component"
}